{
  "term_id": "GO:0005871",
  "gene": "UniProtKB:Q9GZM8",
  "gene_name": "Nuclear distribution protein nudE-like 1",
  "gene_symbol": "NDEL1",
  "term_label": "kinesin complex"
}